{
  "gene_symbol": "SND1-IT1",
  "gene_name": "Uncharacterized protein encoded by SND1-IT1",
  "term_label": "Unknown cellular component",
  "term_id": "UNKNOWN:0003",
  "gene": "UniProtKB:Q9HBX3"
}